{
  "gene": "UniProtKB:Q9NQT4",
  "gene_name": "Exosome complex component RRP46",
  "term_label": "RNA binding",
  "term_id": "GO:0003723",
  "gene_symbol": "EXOSC5"
}